{
  "term_id": "GO:0071013",
  "gene": "UniProtKB:P62316",
  "gene_symbol": "SNRPD2",
  "term_label": "catalytic step 2 spliceosome",
  "gene_name": "Small nuclear ribonucleoprotein Sm D2"
}